{
  "term_label": "protein sequestering activity",
  "gene_symbol": "NFKBIA",
  "term_id": "GO:0140311",
  "gene_name": "NF-kappa-B inhibitor alpha",
  "gene": "UniProtKB:P25963"
}